{
  "gene_name": "Keratin, type I cuticular Ha7",
  "term_label": "keratin filament",
  "gene_symbol": "KRT37",
  "term_id": "GO:0045095",
  "gene": "UniProtKB:O76014"
}